{
  "gene_name": "Synaptojanin-2",
  "gene_symbol": "SYNJ2",
  "term_label": "membrane",
  "term_id": "GO:0016020",
  "gene": "UniProtKB:O15056"
}